negative regulation of T cell apoptotic process [GO:0070233] (biological process) Definition: Any process that stops, prevents, or reduces the frequency, rate or extent of T cell death by apoptotic process. Sources: GOC:add, GOC:mtg_apoptosis, ISBN:0781765196 Also known as: down regulation of T cell apoptosis, down-regulation of T cell apoptosis, downregulation of T cell apoptosis, negative regulation of T lymphocyte apoptosis, negative regulation of T-cell apoptosis, negative regulation of T-lymphocyte apoptosis, negative regulation of programmed cell death of T cells by apoptosis, inhibition of T cell apoptosis, negative regulation of T cell apoptosis Relationships: is a type of negative regulation of lymphocyte apoptotic process [GO:0070229]; is a type of regulation of T cell apoptotic process [GO:0070232]; negatively regulates T cell apoptotic process [GO:0070231] Subtypes: GO:0070236, GO:0070240, negative regulation of thymocyte apoptotic process [GO:0070244], negative regulation of activated CD4-positive, alpha-beta T cell apoptotic process [GO:1905400], GO:1905403